trehalose transport in response to desiccation [GO:0072515] (biological process) Definition: The directed movement of trehalose into, out of or within a cell, or between cells, by means of some agent such as a transporter or pore, that occurs as a result of a desiccation stimulus. A desiccation stimulus signals extreme dryness resulting from the prolonged deprivation of water. Sources: GOC:mah Relationships: is a type of trehalose transport in response to water deprivation [GO:0072514]; is part of cellular response to desiccation [GO:0071465]